{
  "term_id": "GO:0048666",
  "gene": "UniProtKB:P40424",
  "gene_name": "Pre-B-cell leukemia transcription factor 1",
  "term_label": "neuron development",
  "gene_symbol": "PBX1"
}